{
  "gene_name": "Parathyroid hormone 2 receptor",
  "gene": "UniProtKB:P49190",
  "gene_symbol": "PTH2R",
  "term_id": "GO:0007188",
  "term_label": "adenylate cyclase-modulating G protein-coupled receptor signaling pathway"
}